{
  "gene_symbol": "UNC5D",
  "term_label": "axon guidance",
  "term_id": "GO:0007411",
  "gene_name": "Netrin receptor UNC5D",
  "gene": "UniProtKB:Q6UXZ4"
}